regulation of protein localization to cell cortex of cell tip [GO:1990895] (biological process) References: PMID:26150232 Sources: GOC:vw Relationships: is a type of regulation of protein localization to cell tip [GO:1903066]; is_a GO:1904776; regulates protein localization to cell cortex of cell tip [GO:1990896] Definition: Any process that modulates the frequency, rate or extent of protein localization to cell cortex of cell tip. Subtypes: negative regulation of protein localization to cell cortex of cell tip [GO:0106013]